{
  "gene_name": "Cytochrome P450 27C1",
  "term_id": "GO:0061896",
  "term_label": "all-trans retinol 3,4-desaturase activity",
  "gene_symbol": "CYP27C1",
  "gene": "UniProtKB:Q4G0S4"
}